{
  "gene_symbol": "DCAF17",
  "gene": "UniProtKB:Q5H9S7",
  "term_id": "UNKNOWN:0002",
  "gene_name": "DDB1- and CUL4-associated factor 17",
  "term_label": "Unknown biological process"
}